{
  "gene": "UniProtKB:Q8TAF5",
  "term_id": "UNKNOWN:0001",
  "gene_symbol": "FLVCR1-DT",
  "gene_name": "Putative uncharacterized protein LQK1",
  "term_label": "Unknown molecular function"
}